{
  "term_id": "GO:0050660",
  "gene_symbol": "NOS3",
  "gene": "UniProtKB:P29474",
  "term_label": "flavin adenine dinucleotide binding",
  "gene_name": "Nitric oxide synthase 3"
}